histone H4K16 propionyltransferase activity [GO:0141002] (molecular function) Definition: Catalysis of the reaction: histone H4 L-lysine (position 16) + propionyl-CoA = CoA + H+ + histone H3 N6-propionyl-L-lysyl (position 16). Relationships: is a type of GO:0061922 References: PMID:17267393, PMID:29321206, PMID:31794431 Note: Note that the residue position corresponds to the canonical human H4 histone (UniProtKB:P02309); this residue is conserved across all eukaryotes. Note that the initiation methionine is cleaved, so the first residue is S1.